{
  "gene_symbol": "TPM3",
  "term_label": "actin filament binding",
  "gene_name": "Tropomyosin alpha-3 chain",
  "term_id": "GO:0051015",
  "gene": "UniProtKB:P06753"
}